CENP-A containing nucleosome binding [GO:0097030] (molecular function) Also known as: centromere-specific nucleosome binding, centromeric nucleosome binding Definition: Binding to a centromere-specific nucleosome, a form of nucleosome located only at the centromere, in which the histone H3 is replaced by the variant form CENP-A (sometimes known as CenH3). Relationships: is a type of nucleosome binding [GO:0031491] References: PMID:21412236 Sources: GOC:jp